{
  "term_id": "GO:1902711",
  "gene": "UniProtKB:Q8N1C3",
  "gene_symbol": "GABRG1",
  "gene_name": "Gamma-aminobutyric acid receptor subunit gamma-1",
  "term_label": "GABA-A receptor complex"
}